pole plasm oskar mRNA localization [GO:0045451] (biological process) Also known as: establishment and maintenance of oskar mRNA localization in pole plasm, establishment and maintenance of pole plasm oskar mRNA localization, oocyte pole plasm oskar mRNA localization, pole plasm oskar mRNA localisation Regulation: regulated by GO:0007317; negatively regulated by GO:0045855; positively regulated by GO:0045856 Definition: Any process in which oskar mRNA is transported to, or maintained in, the oocyte pole plasm. Relationships: is a type of pole plasm mRNA localization [GO:0019094] Sources: GOC:go_curators